positive regulation of microglia differentiation [GO:0014008] (BP) Also known as: positive regulation of microglial cell differentiation, up regulation of microglia differentiation, up-regulation of microglia differentiation, upregulation of microglia differentiation, activation of microglia differentiation, stimulation of microglia differentiation Sources: GOC:ef Definition: Any process that activates, maintains or increases the frequency, rate or extent of microglia differentiation, the process in which a relatively unspecialized cell acquires specialized features of a microglial cell. Relationships: is a type of regulation of microglia differentiation [GO:0014006]; is a type of positive regulation of macrophage differentiation [GO:0045651]; is a type of GO:0045687; positively regulates microglia differentiation [GO:0014004]